{
  "gene": "UniProtKB:P15151",
  "term_label": "adherens junction",
  "gene_symbol": "PVR",
  "term_id": "GO:0005912",
  "gene_name": "Poliovirus receptor"
}